{
  "term_id": "UNKNOWN:0002",
  "term_label": "Unknown biological process",
  "gene": "UniProtKB:Q96RD2",
  "gene_name": "Olfactory receptor 52B2",
  "gene_symbol": "OR52B2"
}